{
  "gene_name": "Pejvakin",
  "gene_symbol": "PJVK",
  "term_label": "neuronal cell body",
  "term_id": "GO:0043025",
  "gene": "UniProtKB:Q0ZLH3"
}